bacteriocin transmembrane transporter activity [GO:0022885] (molecular function) Relationships: is a type of amide transmembrane transporter activity [GO:0042887]; is a type of GO:0042910; is part of bacteriocin transport [GO:0043213] Definition: Enables the transfer of a bacteriocin from one side of a membrane to the other. Subtypes: colicin transmembrane transporter activity [GO:0042912], GO:0043214 Sources: GOC:mtg_transport, ISBN:0815340729